{
  "gene_name": "Late cornified envelope protein 1C",
  "term_label": "Unknown biological process",
  "gene": "UniProtKB:Q5T751",
  "term_id": "UNKNOWN:0002",
  "gene_symbol": "LCE1C"
}